S100 protein binding [GO:0044548] (molecular function) Sources: GOC:jid Also known as: S100 binding, S100 alpha binding, S100 beta binding Definition: Binding to a S100 protein. S100 is a small calcium and zinc binding protein produced in astrocytes that is implicated in Alzheimer's disease, Down Syndrome and ALS. Relationships: is a type of GO:0005515